mRNA methylguanosine-cap decapping [GO:0110156] (biological process) Subtypes: GO:0000290, deadenylation-independent decapping of nuclear-transcribed mRNA [GO:0031087] Relationships: is a type of mRNA metabolic process [GO:0016071]; is_a RNA decapping [GO:0110154] Definition: Cleavage of the 5'-methylguanosine-cap of an mRNA. The methylguanosine-cap is present at the 5'-end of eukaryotic mRNAs. Decapping inactivates translation initiation and promotes 5'-to-3' decay of mRNA. References: PMID:23287066